{
  "gene_symbol": "RAB3D",
  "term_label": "myosin V binding",
  "gene_name": "Ras-related protein Rab-3D",
  "gene": "UniProtKB:O95716",
  "term_id": "GO:0031489"
}